{
  "gene_name": "Probable ATP-dependent RNA helicase DDX20",
  "gene": "UniProtKB:Q9UHI6",
  "gene_symbol": "DDX20",
  "term_label": "mRNA binding",
  "term_id": "GO:0003729"
}